{
  "gene": "UniProtKB:O14543",
  "term_id": "GO:0046426",
  "term_label": "negative regulation of receptor signaling pathway via JAK-STAT",
  "gene_name": "Suppressor of cytokine signaling 3",
  "gene_symbol": "SOCS3"
}